{
  "gene": "UniProtKB:Q86WV5",
  "term_label": "negative regulation of telomere maintenance via telomerase",
  "gene_symbol": "TEN1",
  "term_id": "GO:0032211",
  "gene_name": "CST complex subunit TEN1"
}